{
  "term_label": "Unknown cellular component",
  "term_id": "UNKNOWN:0003",
  "gene_name": "MKKS centrosomal shuttling protein",
  "gene_symbol": "MKKS",
  "gene": "UniProtKB:V9GZ13"
}